{
  "gene_name": "Cytoplasmic polyadenylation element-binding protein 2",
  "gene": "UniProtKB:Q7Z5Q1",
  "term_id": "GO:0043005",
  "gene_symbol": "CPEB2",
  "term_label": "neuron projection"
}